{
  "gene": "UniProtKB:Q8NEM1",
  "term_label": "RNA polymerase II cis-regulatory region sequence-specific DNA binding",
  "term_id": "GO:0000978",
  "gene_symbol": "ZNF680",
  "gene_name": "Zinc finger protein 680"
}